{
  "term_label": "Unknown biological process",
  "gene_symbol": "SERF2",
  "gene": "UniProtKB:P84101",
  "term_id": "UNKNOWN:0002",
  "gene_name": "Small EDRK-rich factor 2"
}